{
  "term_label": "tRNA (5-carboxymethyluridine(34)-5-O)-methyltransferase activity",
  "gene_name": "Probable tRNA methyltransferase 9B",
  "gene_symbol": "TRMT9B",
  "term_id": "GO:0106335",
  "gene": "UniProtKB:Q9P272"
}